{
  "gene_symbol": "CCL3L1",
  "term_label": "cell chemotaxis",
  "gene_name": "C-C motif chemokine 3-like 1",
  "term_id": "GO:0060326",
  "gene": "UniProtKB:P16619"
}